D1 dopamine receptor binding [GO:0031748] (molecular function) Sources: GOC:mah, GOC:nln Also known as: D1A dopamine receptor binding, D1 dopamine receptor ligand Relationships: is a type of dopamine receptor binding [GO:0050780] Definition: Binding to a D1 dopamine receptor.